{
  "gene_symbol": "APOBEC3A",
  "term_id": "GO:0016554",
  "gene_name": "DNA dC-dU-editing enzyme APOBEC-3A",
  "term_label": "cytidine to uridine editing",
  "gene": "UniProtKB:P31941"
}